{
  "gene_symbol": "CCDC154",
  "term_label": "Unknown molecular function",
  "gene": "UniProtKB:A6NI56",
  "gene_name": "Coiled-coil domain-containing protein 154",
  "term_id": "UNKNOWN:0001"
}